{
  "term_label": "chromatin remodeling",
  "term_id": "GO:0006338",
  "gene_name": "Transcriptional adapter 2-beta",
  "gene": "UniProtKB:Q86TJ2",
  "gene_symbol": "TADA2B"
}